lateral sprouting involved in ureteric bud morphogenesis [GO:0060680] (biological process) References: PMID:16916378 Sources: GOC:dph Relationships: is a type of lateral sprouting from an epithelium [GO:0060601]; is part of GO:0001658 Definition: The process in which a branch forms along the side of a ureteric bud.